cardiac muscle tissue development [GO:0048738] (biological process) Regulation: regulated by regulation of cardiac muscle tissue development [GO:0055024]; positively regulated by GO:0055025; negatively regulated by negative regulation of cardiac muscle tissue development [GO:0055026] Also known as: heart muscle development Sources: GOC:dph, GOC:jid, GOC:lm Definition: The process whose specific outcome is the progression of cardiac muscle over time, from its formation to the mature structure. Relationships: is a type of GO:0014706; is part of GO:0007507 Subtypes: cardiac conduction system development [GO:0003161], atrioventricular node development [GO:0003162], atrial cardiac muscle tissue development [GO:0003228], ventricular cardiac muscle tissue development [GO:0003229]